{
  "term_label": "DNA-binding transcription factor activity",
  "gene_name": "Zinc finger protein 524",
  "gene": "UniProtKB:Q96C55",
  "gene_symbol": "ZNF524",
  "term_id": "GO:0003700"
}